{
  "gene_symbol": "STX7",
  "gene": "UniProtKB:O15400",
  "gene_name": "Syntaxin-7",
  "term_id": "GO:0031201",
  "term_label": "SNARE complex"
}